{
  "term_label": "Unknown molecular function",
  "gene_symbol": "CHRAC1",
  "gene_name": "Chromatin accessibility complex protein 1",
  "gene": "UniProtKB:Q9NRG0",
  "term_id": "UNKNOWN:0001"
}